{
  "term_id": "GO:0005634",
  "gene_symbol": "ZNF875",
  "gene_name": "Zinc finger protein 875",
  "gene": "UniProtKB:P10072",
  "term_label": "nucleus"
}